lipopolysaccharide core region biosynthetic process [GO:0009244] (biological process) Relationships: is a type of GO:0009312; is part of lipopolysaccharide biosynthetic process [GO:0009103] Also known as: LPS core region biosynthetic process, lipopolysaccharide core region anabolism, lipopolysaccharide core region biosynthesis, lipopolysaccharide core region formation, lipopolysaccharide core region synthesis Definition: The chemical reactions and pathways resulting in the formation of the core region of bacterial lipopolysaccharides, which contains ten saccharide residues. Sources: ISBN:0198506732